{
  "gene": "UniProtKB:Q8N1C3",
  "gene_symbol": "GABRG1",
  "term_label": "chloride channel activity",
  "term_id": "GO:0005254",
  "gene_name": "Gamma-aminobutyric acid receptor subunit gamma-1"
}